{
  "term_label": "Unknown cellular component",
  "gene_symbol": "NKAPD1",
  "term_id": "UNKNOWN:0003",
  "gene_name": "Uncharacterized protein NKAPD1",
  "gene": "UniProtKB:Q6ZUT1"
}